{
  "gene": "UniProtKB:P0DUQ2",
  "term_label": "Unknown cellular component",
  "term_id": "UNKNOWN:0003",
  "gene_name": "PRAME family member 9",
  "gene_symbol": "PRAMEF9"
}